regulation of programmed necrotic cell death [GO:0062098] (BP) References: PMID:27258785 Sources: GOC:aruk, GOC:rph Relationships: is a type of GO:0043067; regulates programmed necrotic cell death [GO:0097300] Definition: Any process that modulates the frequency, rate or extent of programmed necrotic cell death. Subtypes: GO:0060544, negative regulation of programmed necrotic cell death [GO:0062099], GO:0062100